{
  "term_label": "Golgi apparatus",
  "gene_name": "N-acetylglucosamine-1-phosphotransferase subunits alpha_beta",
  "term_id": "GO:0005794",
  "gene": "UniProtKB:Q3T906",
  "gene_symbol": "GNPTAB"
}